{
  "gene_symbol": "NOS1",
  "gene_name": "Nitric oxide synthase 1",
  "term_id": "GO:0005829",
  "term_label": "cytosol",
  "gene": "UniProtKB:P29475"
}